{
  "gene": "UniProtKB:A6NHA9",
  "gene_symbol": "OR4C46",
  "gene_name": "Olfactory receptor 4C46",
  "term_label": "Unknown biological process",
  "term_id": "UNKNOWN:0002"
}